cellulosome assembly [GO:0044575] (BP) References: PMID:20373916 Sources: GOC:mengo_curators, GOC:tt Definition: The assembly of a cellulosome, a macromolecular multi-enzyme complex in bacteria that facilitates the breakdown of cellulase, hemicellulase and pectin in the plant cell wall. Regulation: regulated by regulation of cellulosome assembly [GO:1900503]; negatively regulated by negative regulation of cellulosome assembly [GO:1900504]; RO_0002213 by positive regulation of cellulosome assembly [GO:1900505] Relationships: is_a membraneless organelle assembly [GO:0140694]